mitochondrial ADP transmembrane transport [GO:0140021] (biological process) Definition: The process in which ADP is transported across a mitochondrial membrane, into or out of the mitochondrion. References: PMID:2541251 Relationships: is a type of ADP transport [GO:0015866]; is a type of purine-containing compound transmembrane transport [GO:0072530]; is a type of nucleotide transmembrane transport [GO:1901679]